{
  "term_id": "GO:0043484",
  "term_label": "regulation of RNA splicing",
  "gene_name": "AF4_FMR2 family member 2",
  "gene_symbol": "AFF2",
  "gene": "UniProtKB:P51816"
}